{
  "term_label": "isocitrate metabolic process",
  "gene_symbol": "IDH2",
  "gene": "UniProtKB:P48735",
  "term_id": "GO:0006102",
  "gene_name": "Isocitrate dehydrogenase [NADP], mitochondrial"
}